{
  "gene": "UniProtKB:B2RXH2",
  "term_id": "GO:0006338",
  "term_label": "chromatin remodeling",
  "gene_symbol": "KDM4E",
  "gene_name": "Lysine-specific demethylase 4E"
}